{
  "gene": "UniProtKB:O00341",
  "term_label": "neutral L-amino acid transmembrane transporter activity",
  "term_id": "GO:0015175",
  "gene_symbol": "SLC1A7",
  "gene_name": "Excitatory amino acid transporter 5"
}